{
  "term_label": "intracellular sphingolipid homeostasis",
  "gene_symbol": "ORMDL1",
  "gene_name": "ORM1-like protein 1",
  "gene": "UniProtKB:Q9P0S3",
  "term_id": "GO:0090156"
}